{
  "gene_symbol": "ATP11B",
  "term_id": "GO:0045332",
  "gene": "UniProtKB:Q9Y2G3",
  "term_label": "phospholipid translocation",
  "gene_name": "Phospholipid-transporting ATPase IF"
}